{
  "term_label": "translation",
  "gene_name": "Elongation factor 1-alpha 1",
  "gene": "UniProtKB:P68104",
  "term_id": "GO:0006412",
  "gene_symbol": "EEF1A1"
}